{
  "term_id": "GO:0005737",
  "term_label": "cytoplasm",
  "gene_name": "ATP synthase subunit s, mitochondrial",
  "gene": "UniProtKB:Q99766",
  "gene_symbol": "DMAC2L"
}